{
  "gene": "UniProtKB:P01903",
  "gene_name": "HLA class II histocompatibility antigen, DR alpha chain",
  "gene_symbol": "HLA-DRA",
  "term_label": "peptide antigen assembly with MHC class II protein complex",
  "term_id": "GO:0002503"
}